{
  "gene_symbol": "MAN1A2",
  "term_label": "ERAD pathway",
  "term_id": "GO:0036503",
  "gene_name": "Mannosyl-oligosaccharide 1,2-alpha-mannosidase IB",
  "gene": "UniProtKB:O60476"
}